{
  "gene_name": "Adhesion G protein-coupled receptor B1",
  "term_label": "G protein-coupled receptor activity",
  "gene": "UniProtKB:O14514",
  "gene_symbol": "ADGRB1",
  "term_id": "GO:0004930"
}